{
  "term_label": "TORC2 complex",
  "gene_symbol": "PRR5L",
  "term_id": "GO:0031932",
  "gene": "UniProtKB:Q6MZQ0",
  "gene_name": "Proline-rich protein 5-like"
}